long-chain fatty-acyl-CoA biosynthetic process [GO:0035338] (biological process) Note: While there is not universal consensus on the lengths of short-, medium-, long- and very-long-chain fatty acids, the GO uses the definitions in ChEBI (see CHEBI:26666, CHEBI:59554, CHEBI:15904 and CHEBI:27283). Definition: The chemical reactions and pathways resulting in the formation of a long-chain fatty-acyl-CoA any derivative of coenzyme A in which the sulfhydryl group is in a thioester linkage with a long-chain fatty-acyl group. A long-chain fatty acid has an aliphatic tail containing 13 to 22 carbons. Relationships: is a type of GO:0035336; is a type of fatty-acyl-CoA biosynthetic process [GO:0046949] Also known as: long-chain fatty acyl CoA biosynthetic process, long-chain fatty-acyl-CoA anabolism, long-chain fatty-acyl-CoA biosynthesis, long-chain fatty-acyl-CoA formation, long-chain fatty-acyl-CoA synthesis Sources: ISBN:0198506732